{
  "gene_symbol": "DUOX2",
  "gene": "UniProtKB:Q9NRD8",
  "term_label": "superoxide anion generation",
  "gene_name": "Dual oxidase 2",
  "term_id": "GO:0042554"
}